{
  "gene": "UniProtKB:Q16526",
  "gene_name": "Cryptochrome-1",
  "term_label": "negative regulation of DNA-templated transcription",
  "gene_symbol": "CRY1",
  "term_id": "GO:0045892"
}